{
  "gene_name": "LHFPL tetraspan subfamily member 3 protein",
  "gene": "UniProtKB:Q86UP9",
  "term_label": "plasma membrane",
  "gene_symbol": "LHFPL3",
  "term_id": "GO:0005886"
}